2-iminobutanoate deaminase activity [GO:0120242] (molecular function) Definition: Catalysis of the reaction: 2-iminobutanoate + H2O = 2-oxobutanoate + NH4(+). Relationships: is a type of 2-iminobutanoate/2-iminopropanoate deaminase [GO:0120241] Also known as: 2-iminobutanoate/2-iminopropanoate deaminase Sources: RHEA:39975